{
  "term_id": "UNKNOWN:0003",
  "gene_name": "SPRY domain-containing protein 4",
  "gene_symbol": "SPRYD4",
  "term_label": "Unknown cellular component",
  "gene": "UniProtKB:Q8WW59"
}